{
  "gene_name": "Sodium-coupled neutral amino acid symporter 1",
  "gene": "UniProtKB:Q9H2H9",
  "term_label": "glutamine transport",
  "term_id": "GO:0006868",
  "gene_symbol": "SLC38A1"
}